NAADP-sensitive calcium-release channel activity [GO:0072345] (molecular function) Relationships: is a type of intracellularly gated calcium channel activity [GO:0015278] Definition: Enables the transmembrane transfer of a calcium ion by a channel that opens when nicotinic acid adenine dinucleotide phosphate (NAADP) has been bound by the channel complex or one of its constituent parts. References: PMID:19387438, PMID:19557428